{
  "gene": "UniProtKB:Q96B45",
  "gene_name": "BLOC-1-related complex subunit 7",
  "term_id": "UNKNOWN:0001",
  "term_label": "Unknown molecular function",
  "gene_symbol": "BORCS7"
}